positive regulation of myeloid dendritic cell activation [GO:0030887] (biological process) Relationships: is a type of positive regulation of leukocyte activation [GO:0002696]; is a type of regulation of myeloid dendritic cell activation [GO:0030885]; positively regulates myeloid dendritic cell activation [GO:0001773] Also known as: up regulation of myeloid dendritic cell activation, up-regulation of myeloid dendritic cell activation, upregulation of myeloid dendritic cell activation, activation of myeloid dendritic cell activation, stimulation of myeloid dendritic cell activation Definition: Any process that stimulates, induces or increases the rate of myeloid dendritic cell activation. Sources: GOC:mah